regulation of cardiac muscle fiber development [GO:0055018] (BP) Subtypes: GO:0055019, positive regulation of cardiac muscle fiber development [GO:0055020] Also known as: regulation of cardiac muscle fibre development, regulation of heart muscle fiber development Relationships: is a type of GO:0060284; is a type of regulation of cardiac muscle cell differentiation [GO:2000725]; regulates cardiac muscle cell development [GO:0055013] Definition: Any process that modulates the frequency, rate or extent of cardiac muscle fiber development. Sources: GOC:vk